{
  "gene": "UniProtKB:Q03721",
  "gene_name": "Potassium voltage-gated channel subfamily C member 4",
  "gene_symbol": "KCNC4",
  "term_label": "postsynaptic membrane",
  "term_id": "GO:0045211"
}